{
  "term_label": "negative regulation of canonical Wnt signaling pathway",
  "gene": "UniProtKB:O75096",
  "gene_symbol": "LRP4",
  "term_id": "GO:0090090",
  "gene_name": "Low-density lipoprotein receptor-related protein 4"
}